{
  "gene_name": "Histone-lysine N-methyltransferase SETD2",
  "gene": "UniProtKB:Q9BYW2",
  "term_id": "GO:0005634",
  "gene_symbol": "SETD2",
  "term_label": "nucleus"
}